{
  "term_label": "G protein-coupled receptor signaling pathway",
  "gene": "UniProtKB:Q9P2W3",
  "gene_name": "Guanine nucleotide-binding protein G(I)_G(S)_G(O) subunit gamma-13",
  "term_id": "GO:0007186",
  "gene_symbol": "GNG13"
}